{
  "gene": "UniProtKB:P08133",
  "gene_name": "Annexin A6",
  "term_label": "vesicle membrane",
  "term_id": "GO:0012506",
  "gene_symbol": "ANXA6"
}